{
  "gene_name": "Acyl-coenzyme A thioesterase 8",
  "term_id": "GO:0009062",
  "gene": "UniProtKB:O14734",
  "gene_symbol": "ACOT8",
  "term_label": "fatty acid catabolic process"
}